{
  "term_label": "Unknown biological process",
  "gene": "UniProtKB:Q8NDZ6",
  "gene_name": "Transmembrane protein 161B",
  "term_id": "UNKNOWN:0002",
  "gene_symbol": "TMEM161B"
}